{
  "term_id": "UNKNOWN:0003",
  "gene_name": "Thyroxine 5-deiodinase",
  "term_label": "Unknown cellular component",
  "gene": "UniProtKB:P55073",
  "gene_symbol": "DIO3"
}